{
  "term_label": "cellular senescence",
  "gene_symbol": "HRAS",
  "gene": "UniProtKB:P01112",
  "gene_name": "GTPase HRas",
  "term_id": "GO:0090398"
}